leucoplast stroma [GO:0009576] (cellular component) Relationships: is a type of GO:0009532; is part of leucoplast [GO:0009516] Sources: GOC:mah Definition: The space enclosed by the double membrane of a leucoplast.